{
  "gene": "UniProtKB:Q8TDC3",
  "gene_name": "Serine_threonine-protein kinase BRSK1",
  "gene_symbol": "BRSK1",
  "term_label": "axonogenesis",
  "term_id": "GO:0007409"
}